{
  "term_label": "plasma membrane",
  "gene_symbol": "KIR2DL1",
  "gene_name": "Killer cell immunoglobulin-like receptor 2DL1",
  "term_id": "GO:0005886",
  "gene": "UniProtKB:P43626"
}